{
  "gene_symbol": "ZNF362",
  "term_label": "DNA-binding transcription factor activity",
  "term_id": "GO:0003700",
  "gene_name": "Zinc finger protein 362",
  "gene": "UniProtKB:Q5T0B9"
}